{
  "term_label": "cysteine-type deubiquitinase activity",
  "gene_symbol": "OTUB2",
  "gene": "UniProtKB:Q96DC9",
  "gene_name": "Ubiquitin thioesterase OTUB2",
  "term_id": "GO:0004843"
}